{
  "gene_symbol": "SMURF1",
  "term_id": "GO:0046332",
  "gene": "UniProtKB:Q9HCE7",
  "term_label": "SMAD binding",
  "gene_name": "E3 ubiquitin-protein ligase SMURF1"
}